{
  "term_label": "BLOC-3 complex",
  "term_id": "GO:0031085",
  "gene_symbol": "HPS4",
  "gene": "UniProtKB:Q9NQG7",
  "gene_name": "BLOC-3 complex member HPS4"
}